{
  "gene_symbol": "HMGCS2",
  "gene": "UniProtKB:P54868",
  "gene_name": "Hydroxymethylglutaryl-CoA synthase, mitochondrial",
  "term_label": "farnesyl diphosphate biosynthetic process, mevalonate pathway",
  "term_id": "GO:0010142"
}